{
  "term_id": "GO:0005615",
  "gene_name": "Lactoperoxidase",
  "term_label": "extracellular space",
  "gene_symbol": "LPO",
  "gene": "UniProtKB:P22079"
}